male meiosis cytokinesis [GO:0007112] (biological process) Sources: GOC:ai Relationships: is a type of meiotic cytokinesis [GO:0033206]; is part of GO:0007140 Also known as: cytokinesis after male meiosis, cytokinesis involved in male meiotic cell cycle Definition: A cell cycle process that occurs as part of the male meiotic cell cycle and results in the division of the cytoplasm of a cell to produce two daughter cells.